bone development [GO:0060348] (biological process) Sources: GOC:dph Regulation: regulated by regulation of bone development [GO:1903010]; negatively regulated by GO:1903011; positively regulated by GO:1903012 Relationships: is a type of animal organ development [GO:0048513]; is part of skeletal system development [GO:0001501] Definition: The process whose specific outcome is the progression of bone over time, from its formation to the mature structure. Bone is the hard skeletal connective tissue consisting of both mineral and cellular components.